{
  "term_label": "nuclear localization sequence binding",
  "term_id": "GO:0008139",
  "gene": "UniProtKB:Q96HA1",
  "gene_symbol": "POM121",
  "gene_name": "Nuclear envelope pore membrane protein POM 121"
}